{
  "gene_symbol": "A8MWL6",
  "term_id": "UNKNOWN:0002",
  "gene_name": "Putative synaptogyrin-2 like protein",
  "term_label": "Unknown biological process",
  "gene": "UniProtKB:A8MWL6"
}